{
  "gene_symbol": "ST6GALNAC3",
  "term_id": "GO:0001665",
  "gene_name": "Alpha-N-acetylgalactosaminide alpha-2,6-sialyltransferase 3",
  "term_label": "alpha-N-acetylgalactosaminide alpha-2,6-sialyltransferase activity",
  "gene": "UniProtKB:Q8NDV1"
}